interleukin-32-mediated signaling pathway [GO:0097399] (biological process) Also known as: IL-32-mediated signaling pathway, IL-32-mediated signalling pathway, interleukin-32-mediated signalling pathway References: PMID:21602493 Sources: GOC:ic Relationships: is a type of cytokine-mediated signaling pathway [GO:0019221]; is part of cellular response to interleukin-32 [GO:0097397] Definition: The series of molecular signals initiated by interleukin-32 binding to its receptor on the surface of a target cell, and ending with the regulation of a downstream cellular process, e.g. transcription.